lipid antigen transport [GO:0002494] (biological process) Relationships: is a type of lipid transport [GO:0006869]; is part of antigen processing and presentation of lipid antigen via MHC class Ib [GO:0048003] References: PMID:15928678, PMID:15928680 Sources: GOC:add Definition: The directed movement of a lipid antigen into, out of or within a cell, or between cells, by means of some agent such as a transporter or pore.